{
  "gene_symbol": "PALLD",
  "gene": "UniProtKB:Q8WX93",
  "term_label": "Z disc",
  "gene_name": "Palladin",
  "term_id": "GO:0030018"
}